regulation of blood vessel endothelial cell differentiation [GO:0110057] (biological process) Definition: Any process that modulates the frequency, rate or extent of blood vessel endothelial cell differentiation. References: PMID:23072816 Sources: GOC:BHF, GOC:BHF_miRNA, GOC:rph Subtypes: positive regulation of blood vessel endothelial cell differentiation [GO:0110058], negative regulation of blood vessel endothelial cell differentiation [GO:0110059], GO:2000787 Relationships: is a type of regulation of endothelial cell differentiation [GO:0045601]; regulates blood vessel endothelial cell differentiation [GO:0060837]